{
  "gene": "UniProtKB:Q96Q07",
  "gene_symbol": "BTBD9",
  "term_label": "circadian behavior",
  "gene_name": "BTB_POZ domain-containing protein 9",
  "term_id": "GO:0048512"
}